regulation of endosomal vesicle fusion [GO:1905364] (biological process) Definition: Any process that modulates the frequency, rate or extent of endosomal vesicle fusion. Relationships: is a type of regulation of vesicle fusion [GO:0031338]; regulates endosomal vesicle fusion [GO:0034058] Also known as: regulation of endosome vesicle fusion Subtypes: negative regulation of endosomal vesicle fusion [GO:1905362], positive regulation of endosomal vesicle fusion [GO:1905363] References: PMID:26911690 Sources: GOC:PARL, GOC:TermGenie, GOC:bc, GO_REF:0000058